ornithine metabolic process [GO:0006591] (biological process) Also known as: ornithine metabolism Definition: The chemical reactions and pathways involving ornithine, an amino acid only rarely found in proteins, but which is important in living organisms as an intermediate in the reactions of the urea cycle and in arginine biosynthesis. Regulation: regulated by regulation of ornithine metabolic process [GO:0090368] Sources: GOC:jl, ISBN:0192801023 Subtypes: ornithine biosynthetic process [GO:0006592], L-ornithine catabolic process [GO:0006593], L-alanine biosynthetic process via ornithine [GO:0019273], L-glutamate catabolic process to ornithine [GO:0019555] Relationships: is a type of non-proteinogenic amino acid metabolic process [GO:0170041]; is a type of alpha-amino acid metabolic process [GO:1901605]